{
  "gene": "UniProtKB:Q9Y6P5",
  "term_label": "positive regulation of macroautophagy",
  "term_id": "GO:0016239",
  "gene_name": "Sestrin-1",
  "gene_symbol": "SESN1"
}